{
  "gene_symbol": "TMEM239",
  "term_id": "UNKNOWN:0002",
  "gene_name": "Transmembrane protein 239",
  "gene": "UniProtKB:Q8WW34",
  "term_label": "Unknown biological process"
}